{
  "gene": "UniProtKB:Q92503",
  "gene_symbol": "SEC14L1",
  "term_label": "RIG-I binding",
  "gene_name": "SEC14-like protein 1",
  "term_id": "GO:0039552"
}